smooth endoplasmic reticulum calcium ion homeostasis [GO:0051563] (biological process) Definition: Any process involved in the maintenance of an internal steady state of calcium ions within the smooth endoplasmic reticulum of a cell or between the smooth endoplasmic reticulum and its surroundings. Relationships: is a type of endoplasmic reticulum calcium ion homeostasis [GO:0032469]; occurs in smooth endoplasmic reticulum [GO:0005790] Sources: GOC:ai, GOC:mah Also known as: calcium ion homeostasis in smooth ER, calcium ion homeostasis in smooth endoplasmic reticulum, regulation of calcium ion concentration in smooth ER, regulation of calcium ion concentration in smooth endoplasmic reticulum, regulation of smooth ER calcium ion concentration, regulation of smooth endoplasmic reticulum calcium ion concentration, smooth ER calcium ion concentration regulation, smooth ER calcium ion homeostasis, smooth endoplasmic reticulum calcium ion concentration regulation Subtypes: positive regulation of smooth endoplasmic reticulum calcium ion concentration [GO:0051564], GO:0051565